{
  "gene_name": "Glutamate receptor ionotropic, delta-2",
  "term_label": "AMPA glutamate receptor complex",
  "gene_symbol": "GRID2",
  "gene": "UniProtKB:O43424",
  "term_id": "GO:0032281"
}